{
  "gene": "UniProtKB:Q9H211",
  "term_id": "GO:0000076",
  "gene_name": "DNA replication factor Cdt1",
  "term_label": "DNA replication checkpoint signaling",
  "gene_symbol": "CDT1"
}